{
  "term_id": "UNKNOWN:0003",
  "gene_symbol": "PEBP1",
  "gene_name": "Phosphatidylethanolamine-binding protein 1",
  "gene": "UniProtKB:P30086",
  "term_label": "Unknown cellular component"
}